{
  "term_id": "GO:0005789",
  "gene_symbol": "CALR",
  "term_label": "endoplasmic reticulum membrane",
  "gene_name": "Calreticulin",
  "gene": "UniProtKB:P27797"
}